pronephric nephron morphogenesis [GO:0039007] (biological process) Definition: The process in which the anatomical structures of the pronephric nephron are generated and organized. A pronephric nephron is the functional unit of the pronephros. Relationships: is a type of nephron morphogenesis [GO:0072028]; is part of pronephric nephron development [GO:0039019]; is part of pronephros morphogenesis [GO:0072114] Sources: GOC:mtg_kidney_jan10